{
  "gene": "UniProtKB:Q8IZS5",
  "term_id": "UNKNOWN:0003",
  "term_label": "Unknown cellular component",
  "gene_symbol": "OFCC1",
  "gene_name": "Orofacial cleft 1 candidate gene 1 protein"
}